{
  "gene": "UniProtKB:Q9BUH8",
  "gene_name": "Brain-enriched guanylate kinase-associated protein",
  "term_label": "synapse",
  "term_id": "GO:0045202",
  "gene_symbol": "BEGAIN"
}